{
  "term_id": "GO:0005829",
  "gene": "UniProtKB:Q96S44",
  "term_label": "cytosol",
  "gene_name": "EKC_KEOPS complex subunit TP53RK",
  "gene_symbol": "TP53RK"
}